interleukin-2-mediated signaling pathway [GO:0038110] (biological process) Sources: GOC:nhn, GOC:signaling Relationships: is a type of cytokine-mediated signaling pathway [GO:0019221]; is part of GO:0071352 Also known as: IL-2-mediated signaling pathway, interleukin-2-mediated signalling pathway Regulation: regulated by regulation of interleukin-2-mediated signaling pathway [GO:1902205]; negatively regulated by negative regulation of interleukin-2-mediated signaling pathway [GO:1902206]; RO_0002213 by positive regulation of interleukin-2-mediated signaling pathway [GO:1902207] Definition: The series of molecular signals initiated by interleukin-2 binding to its receptor on the surface of a cell, and ending with the regulation of a downstream cellular process, e.g. transcription.